{
  "gene_name": "Zinc finger protein 585A",
  "term_label": "transcription cis-regulatory region binding",
  "gene": "UniProtKB:Q6P3V2",
  "term_id": "GO:0000976",
  "gene_symbol": "ZNF585A"
}